{
  "gene": "UniProtKB:Q9UJJ9",
  "term_id": "GO:0005794",
  "gene_symbol": "GNPTG",
  "gene_name": "N-acetylglucosamine-1-phosphotransferase subunit gamma",
  "term_label": "Golgi apparatus"
}